Scc2-Scc4 cohesin loading complex [GO:0090694] (cellular component) Definition: A eukaryotically conserved heterodimeric protein complex (comprising adherin and the chromatid cohesion factor MAU2/Scc4/Ssl3) required for the loading of a cohesin, complex onto DNA. Relationships: is a type of SMC loading complex [GO:0032116] References: PMID:24291789 Sources: GOC:vw Also known as: Mis4-Ssl3 cohesin loading complex